regulation of cellular senescence [GO:2000772] (BP) Relationships: is a type of regulation of cellular process [GO:0050794]; regulates cellular senescence [GO:0090398] Definition: Any process that modulates the frequency, rate or extent of cellular senescence. Subtypes: negative regulation of cellular senescence [GO:2000773], positive regulation of cellular senescence [GO:2000774] Sources: GOC:BHF